{
  "gene_name": "Calcium permeable stress-gated cation channel 1",
  "term_id": "GO:0005886",
  "gene": "UniProtKB:Q9P1W3",
  "term_label": "plasma membrane",
  "gene_symbol": "TMEM63C"
}